peptidoglycan turnover [GO:0009254] (biological process) Definition: The continual breakdown and regeneration of peptidoglycan required to maintain the bacterial cell wall. Peptidoglycans consist of long glycan strands of alternating residues of beta-(1,4) linked N-acetylglucosamine and N-acetylmuramic acid, cross-linked by short peptides. Also known as: murein turnover References: PMID:31296364 Relationships: is a type of GO:0000270